sucrose synthase activity [GO:0016157] (molecular function) Also known as: NDP-glucose:D-fructose 2-alpha-D-glucosyltransferase activity, UDP-glucose-fructose glucosyltransferase activity, UDPglucose-fructose glucosyltransferase activity, sucrose synthetase activity, sucrose-UDP glucosyltransferase activity, sucrose-uridine diphosphate glucosyltransferase activity, uridine diphosphoglucose-fructose glucosyltransferase activity Relationships: is a type of UDP-glucosyltransferase activity [GO:0035251] Definition: Catalysis of the reaction: an NDP-alpha-D-glucose + D-fructose = a ribonucleoside 5'-diphosphate + H+ + sucrose. The phosphate acceptor can be UDP or ADP. Sources: RHEA:16241